{
  "gene_name": "Zinc finger protein 671",
  "term_label": "DNA-binding transcription factor activity",
  "term_id": "GO:0003700",
  "gene_symbol": "ZNF671",
  "gene": "UniProtKB:Q8TAW3"
}